{
  "gene_symbol": "HAX1",
  "term_id": "GO:0016324",
  "gene": "UniProtKB:O00165",
  "gene_name": "HCLS1-associated protein X-1",
  "term_label": "apical plasma membrane"
}